negative regulation of oocyte development [GO:0060283] (biological process) Sources: GOC:dph, GOC:tb Definition: Any process that decreases the rate or extent of the process whose specific outcome is the progression of an oocyte over time, from initial commitment of the cell to its specific fate, to the fully functional differentiated cell. Relationships: is a type of GO:0010721; is a type of regulation of oocyte development [GO:0060281]; is a type of GO:2000242; negatively regulates GO:0048599